nicotinate transport [GO:2001142] (biological process) Definition: The directed movement of a nicotinateacetate into, out of or within a cell, or between cells, by means of some agent such as a transporter or pore. Relationships: is a type of GO:0015718; is a type of nitrogen compound transport [GO:0071705] Sources: GOC:obol